outer ear emergence [GO:0060186] (biological process) Definition: The growth of the outer ear. Relationships: is a type of developmental growth involved in morphogenesis [GO:0060560]; is part of outer ear morphogenesis [GO:0042473] Sources: GOC:dph Also known as: ear elevation, ear extroversion, outer ear growth